{
  "term_label": "Unknown molecular function",
  "gene_name": "Leucine zipper putative tumor suppressor 3",
  "gene_symbol": "LZTS3",
  "term_id": "UNKNOWN:0001",
  "gene": "UniProtKB:O60299"
}